ACG codon-amino acid adaptor activity [GO:0033440] (molecular function) Definition: A triplet codon-amino acid adaptor activity that recognizes an ACG codon. Also known as: threonine tRNA Note: Note that in the standard genetic code, ACG codes for threonine. Relationships: is a type of triplet codon-amino acid adaptor activity [GO:0030533] Sources: GOC:mah